{
  "gene": "UniProtKB:P12004",
  "term_label": "PCNA complex",
  "gene_symbol": "PCNA",
  "gene_name": "Proliferating cell nuclear antigen",
  "term_id": "GO:0043626"
}